{
  "gene_symbol": "TPCN2",
  "gene_name": "Two pore channel protein 2",
  "term_label": "endocytosis involved in viral entry into host cell",
  "term_id": "GO:0075509",
  "gene": "UniProtKB:Q8NHX9"
}